{
  "gene": "UniProtKB:Q14573",
  "term_label": "sarcoplasmic reticulum",
  "gene_name": "Inositol 1,4,5-trisphosphate receptor type 3",
  "gene_symbol": "ITPR3",
  "term_id": "GO:0016529"
}